{
  "term_label": "Unknown biological process",
  "gene_symbol": "C1QTNF5",
  "gene": "UniProtKB:Q9BXJ0",
  "term_id": "UNKNOWN:0002",
  "gene_name": "Complement C1q tumor necrosis factor-related protein 5"
}